{
  "gene_name": "Uncharacterized protein C4orf3",
  "gene_symbol": "C4orf3",
  "term_label": "Unknown biological process",
  "gene": "UniProtKB:Q8WVX3",
  "term_id": "UNKNOWN:0002"
}